dimethyl ether metabolic process [GO:0018905] (BP) Also known as: dimethyl ether metabolism, methyl ether metabolic process, methyl ether metabolism Sources: UM-BBD_pathwayID:dme Definition: The chemical reactions and pathways involving dimethyl ether, CH3-O-CH3, the simplest ether. Dimethyl ether, also known wood ether and methyl ether, is a colorless gas that has been used in refrigeration applications. Relationships: is a type of xenobiotic metabolic process [GO:0006805]